{
  "gene_name": "Variable charge X-linked protein 2",
  "gene": "UniProtKB:Q9H322",
  "gene_symbol": "VCX2",
  "term_label": "brain development",
  "term_id": "GO:0007420"
}